{
  "gene": "UniProtKB:Q7Z6Z7",
  "gene_name": "E3 ubiquitin-protein ligase HUWE1",
  "term_id": "GO:0007030",
  "term_label": "Golgi organization",
  "gene_symbol": "HUWE1"
}